{
  "gene": "UniProtKB:Q9BVQ7",
  "term_label": "ATP hydrolysis activity",
  "gene_name": "ATPase family gene 2 protein homolog B",
  "term_id": "GO:0016887",
  "gene_symbol": "AFG2B"
}